oligosaccharyltransferase complex [GO:0008250] (cellular component) Also known as: OST complex, oligosaccharyl transferase complex, OSTCI, OSTCII, OSTCIII Definition: A protein complex that is found in the endoplasmic reticulum membrane of eukaryotes and transfers lipid-linked oligosaccharide precursor to asparagine residues on nascent proteins. The complex includes at least eight non-identical subunits. Different forms of the complex containing distinct subunits have been detected in mammals. References: PMID:15835887, PMID:31810196, PMID:32316603 Relationships: is_a membrane protein complex [GO:0098796]; is a type of endoplasmic reticulum protein-containing complex [GO:0140534]; is a type of transferase complex [GO:1990234]; is part of endoplasmic reticulum membrane [GO:0005789] Subtypes: GO:0160226, oligosaccharyltransferase complex B [GO:0160227]